{
  "term_label": "Unknown molecular function",
  "gene_name": "Suppressor of fused homolog",
  "gene_symbol": "SUFU",
  "term_id": "UNKNOWN:0001",
  "gene": "UniProtKB:Q9UMX1"
}